{
  "gene_symbol": "POLR2H",
  "gene": "UniProtKB:P52434",
  "term_id": "GO:0005666",
  "term_label": "RNA polymerase III complex",
  "gene_name": "DNA-directed RNA polymerases I, II, and III subunit RPABC3"
}